{
  "term_label": "nucleus",
  "term_id": "GO:0005634",
  "gene_symbol": "PTP4A2",
  "gene": "UniProtKB:Q12974",
  "gene_name": "Protein tyrosine phosphatase type IVA 2"
}